{
  "term_id": "GO:0043066",
  "gene_name": "E3 ubiquitin-protein ligase Mdm2",
  "gene": "UniProtKB:Q00987",
  "term_label": "negative regulation of apoptotic process",
  "gene_symbol": "MDM2"
}